{
  "term_id": "UNKNOWN:0002",
  "term_label": "Unknown biological process",
  "gene": "UniProtKB:Q12765",
  "gene_name": "Secernin-1",
  "gene_symbol": "SCRN1"
}